Notch signaling pathway involved in somitogenesis [GO:1902359] (biological process) Definition: Any Notch signaling pathway that is involved in somitogenesis. Relationships: is a type of Notch signaling pathway [GO:0007219]; is part of GO:0001756 References: PMID:21795391 Sources: GOC:TermGenie, GOC:dph Regulation: regulated by regulation of Notch signaling pathway involved in somitogenesis [GO:1902366]; RO_0002212 by negative regulation of Notch signaling pathway involved in somitogenesis [GO:1902367] Also known as: N signaling pathway involved in formation of mesodermal clusters, N signaling pathway involved in somitogenesis, N signalling pathway involved in formation of mesodermal clusters, N signalling pathway involved in somitogenesis, Notch receptor signaling pathway involved in formation of mesodermal clusters, Notch receptor signaling pathway involved in somitogenesis, Notch receptor signalling pathway involved in formation of mesodermal clusters, Notch receptor signalling pathway involved in somitogenesis, Notch signaling pathway involved in formation of mesodermal clusters, Notch signalling pathway involved in formation of mesodermal clusters, Notch signalling pathway involved in somitogenesis, Notch-receptor signaling pathway involved in formation of mesodermal clusters, Notch-receptor signaling pathway involved in somitogenesis, Notch-receptor signalling pathway involved in formation of mesodermal clusters, Notch-receptor signalling pathway involved in somitogenesis